cellular response to sulfur starvation [GO:0010438] (biological process) Definition: Any process that results in a change in state or activity of a cell (in terms of movement, secretion, enzyme production, gene expression, etc.) as a result of deprivation of sulfur. Relationships: is a type of cellular response to starvation [GO:0009267] References: PMID:17420480